{
  "gene": "UniProtKB:P15407",
  "term_label": "RNA polymerase II cis-regulatory region sequence-specific DNA binding",
  "term_id": "GO:0000978",
  "gene_symbol": "FOSL1",
  "gene_name": "Fos-related antigen 1"
}